{
  "gene_symbol": "ARL5C",
  "gene": "UniProtKB:A6NH57",
  "term_id": "GO:0016192",
  "term_label": "vesicle-mediated transport",
  "gene_name": "Putative ADP-ribosylation factor-like protein 5C"
}